terrein biosynthetic process [GO:0140880] (biological process) Relationships: is a type of mycotoxin biosynthetic process [GO:0043386]; is a type of GO:0046173 Definition: The chemical reactions and pathways resulting in the formation of terrein, a fungal metabolite with ecological, antimicrobial, antiproliferative, and antioxidative activities. References: PMID:24816227 Also known as: terrein anabolism, terrein biosynthesis, terrein formation, terrein synthesis Regulation: positively regulated by positive regulation terrein biosynthetic process [GO:0140881]